positive regulation of toll-like receptor 4 signaling pathway [GO:0034145] (biological process) Definition: Any process that activates or increases the frequency, rate, or extent of toll-like receptor 4 signaling pathway. References: PMID:16551253, PMID:17328678 Sources: GOC:add Relationships: is a type of regulation of toll-like receptor 4 signaling pathway [GO:0034143]; is a type of positive regulation of pattern recognition receptor signaling pathway [GO:0062208]; positively regulates toll-like receptor 4 signaling pathway [GO:0034142] Also known as: positive regulation of TLR4 signaling pathway, positive regulation of toll-like receptor 4 signalling pathway